positive regulation of cholangiocyte apoptotic process [GO:1904194] (biological process) Relationships: is a type of positive regulation of epithelial cell apoptotic process [GO:1904037]; is a type of GO:1904192; positively regulates GO:1902488 Definition: Any process that activates or increases the frequency, rate or extent of cholangiocyte apoptotic process. References: PMID:24498161 Sources: GOC:TermGenie, GO_REF:0000058 Also known as: positive regulation of epithelial cell of bile duct apoptotic process, up regulation of cholangiocyte apoptotic process, up regulation of epithelial cell of bile duct apoptotic process, up-regulation of cholangiocyte apoptotic process, up-regulation of epithelial cell of bile duct apoptotic process, upregulation of cholangiocyte apoptotic process, upregulation of epithelial cell of bile duct apoptotic process, activation of cholangiocyte apoptosis, activation of cholangiocyte apoptotic process, activation of epithelial cell of bile duct apoptosis, activation of epithelial cell of bile duct apoptotic process, positive regulation of cholangiocyte apoptosis, positive regulation of epithelial cell of bile duct apoptosis, up regulation of cholangiocyte apoptosis, up regulation of epithelial cell of bile duct apoptosis, up-regulation of cholangiocyte apoptosis, up-regulation of epithelial cell of bile duct apoptosis, upregulation of cholangiocyte apoptosis, upregulation of epithelial cell of bile duct apoptosis